thioglucosidase activity [GO:0019137] (molecular function) Definition: Catalysis of the reaction: a thioglucoside + H2O = a thiol + a sugar. Sources: EC:3.2.1.147 Also known as: myrosinase activity, sinigrase activity, sinigrinase activity, thioglucoside glucohydrolase activity Relationships: is a type of GO:0004553